{
  "gene_symbol": "FBXO45",
  "gene_name": "F-box_SPRY domain-containing protein 1",
  "gene": "UniProtKB:P0C2W1",
  "term_label": "proteasome-mediated ubiquitin-dependent protein catabolic process",
  "term_id": "GO:0043161"
}